{
  "gene_symbol": "PCBP4",
  "gene_name": "Poly(rC)-binding protein 4",
  "term_id": "GO:0003729",
  "term_label": "mRNA binding",
  "gene": "UniProtKB:P57723"
}